{
  "gene_name": "Transmembrane protein 18",
  "term_label": "nuclear membrane",
  "term_id": "GO:0031965",
  "gene": "UniProtKB:Q96B42",
  "gene_symbol": "TMEM18"
}